4-hydroxymuconic-semialdehyde dehydrogenase activity [GO:0018481] (molecular function) Definition: Catalysis of the reaction: <stereo>cis,trans</stereo>-4-hydroxymuconate semialdehyde + H2O + NAD+ = 2 H+ + maleylacetate + NADH. Also known as: 4-hydroxymuconic-semialdehyde:NAD+ oxidoreductase activity Relationships: is a type of oxidoreductase activity, acting on the aldehyde or oxo group of donors, NAD or NADP as acceptor [GO:0016620] Sources: EC:1.2.1.61, RHEA:22420